{
  "gene_symbol": "BCL7C",
  "term_label": "Unknown cellular component",
  "term_id": "UNKNOWN:0003",
  "gene": "UniProtKB:Q8WUZ0",
  "gene_name": "B-cell CLL_lymphoma 7 protein family member C"
}